{
  "gene_name": "Disintegrin and metalloproteinase domain-containing protein 15",
  "term_label": "metalloendopeptidase activity",
  "gene_symbol": "ADAM15",
  "term_id": "GO:0004222",
  "gene": "UniProtKB:Q13444"
}